{
  "term_id": "GO:0005737",
  "gene_name": "Inhibitor of nuclear factor kappa-B kinase subunit beta",
  "term_label": "cytoplasm",
  "gene": "UniProtKB:O14920",
  "gene_symbol": "IKBKB"
}